{
  "gene": "UniProtKB:Q30KR1",
  "term_label": "CCR6 chemokine receptor binding",
  "term_id": "GO:0031731",
  "gene_name": "Putative beta-defensin 109B",
  "gene_symbol": "DEFB109B"
}